{
  "gene_symbol": "ESX1",
  "term_label": "DNA-binding transcription factor activity, RNA polymerase II-specific",
  "term_id": "GO:0000981",
  "gene_name": "Homeobox protein ESX1",
  "gene": "UniProtKB:Q8N693"
}